response to organophosphorus [GO:0046683] (biological process) Subtypes: response to ATP [GO:0033198], response to cAMP [GO:0051591], response to cGMP [GO:0070305], GO:0080094, response to 2-O-acetyl-1-O-hexadecyl-sn-glycero-3-phosphocholine [GO:1904316], response to 1-oleoyl-sn-glycerol 3-phosphate [GO:1904565], response to phosphatidylethanolamine [GO:1905711], GO:1905834 Sources: ISBN:0721662544 Definition: Any process that results in a change in state or activity of a cell or an organism (in terms of movement, secretion, enzyme production, gene expression, etc.) as a result of an organophosphorus stimulus. Organophosphorus is a compound containing phosphorus bound to an organic molecule; several organophosphorus compounds are used as insecticides, and they are highly toxic cholinesterase inhibitors. Relationships: is a type of response to chemical [GO:0042221] Also known as: organophosphorus resistance, organophosphorus susceptibility/resistance